extraction of mislocalized protein from mitochondrial outer membrane [GO:0140570] (biological process) Definition: The removal of a mislocalized protein from the mitochondrial outer membrane. References: PMID:32973005 Also known as: extraction of mislocalized protein from outer mitochondrion membrane Relationships: is a type of extraction of mislocalized protein from membrane [GO:0140568]